regulation of interleukin-2-mediated signaling pathway [GO:1902205] (biological process) Also known as: regulation of IL-2-mediated signaling pathway, regulation of interleukin-2-mediated signalling pathway Subtypes: GO:1902206, positive regulation of interleukin-2-mediated signaling pathway [GO:1902207] Relationships: is a type of regulation of cytokine-mediated signaling pathway [GO:0001959]; regulates interleukin-2-mediated signaling pathway [GO:0038110] References: PMID:11909529 Sources: GOC:TermGenie Definition: Any process that modulates the frequency, rate or extent of interleukin-2-mediated signaling pathway.